{
  "gene": "UniProtKB:P11215",
  "term_id": "GO:0007229",
  "gene_symbol": "ITGAM",
  "gene_name": "Integrin alpha-M",
  "term_label": "integrin-mediated signaling pathway"
}